molecular carrier activity [GO:0140104] (molecular function) Definition: Directly binding to a specific ion or molecule and delivering it either to an acceptor molecule or to a specific location. Sources: GOC:molecular_function_refactoring, GOC:pdt Note: Note that a carrier moves with its substrate/cargo, while a transporter does not move with the cargo, but facilitates the change in localization. Relationships: is a type of molecular_function [GO:0003674]; has part GO:0005488 Subtypes: oxygen carrier activity [GO:0005344], metallochaperone activity [GO:0016530], sulfur carrier activity [GO:0097163], nucleocytoplasmic carrier activity [GO:0140142], GO:0140414, protein carrier chaperone [GO:0140597]